calcium ion binding involved in regulation of presynaptic cytosolic calcium ion concentration [GO:0099534] (molecular function) Relationships: is a type of calcium ion binding involved in regulation of cytosolic calcium ion concentration [GO:0099510]; is part of regulation of presynaptic cytosolic calcium ion concentration [GO:0099509]; occurs in presynaptic cytosol [GO:0099523] References: PMID:24442513, PMID:26190970 Definition: The directed change of presynaptic cytosolic free calcium ion concentration in the cytosol via the reversible binding of calcium ions to calcium-binding proteins in the cytosol thereby modulating the spatial and temporal dynamics of changes in presynaptic cytosolic calcium concentrations. Also known as: calcium ion binding involved in regulation of presynaptic cytosolic calcium levels, presynaptic calcium ion buffering, regulation of presynaptic cytosolic calcium ion concentration by calcium ion buffering